post-embryonic cardiac muscle cell growth involved in heart morphogenesis [GO:0003247] (biological process) Definition: The growth of a cardiac muscle cell during the postembryonic period that contributes to the shaping of the heart. Sources: GOC:mtg_heart Relationships: is a type of growth involved in heart morphogenesis [GO:0003241]; is a type of GO:0048588; is part of cardiac muscle tissue growth involved in heart morphogenesis [GO:0003245]